{
  "gene_name": "Membrane-bound transcription factor site-1 protease",
  "gene": "UniProtKB:Q14703",
  "term_label": "Golgi apparatus",
  "gene_symbol": "MBTPS1",
  "term_id": "GO:0005794"
}